aminoacylase activity [GO:0004046] (molecular function) Relationships: is a type of hydrolase activity, acting on carbon-nitrogen (but not peptide) bonds, in linear amides [GO:0016811] Sources: EC:3.5.1.14 Definition: Catalysis of the reaction: an N-acyl-L-amino acid + H2O = a carboxylate + an L-amino acid. Also known as: acylase I activity, aminoacylase I activity, dehydropeptidase II activity, L-amino-acid acylase activity, L-aminoacylase activity, N-acyl-L-amino-acid amidohydrolase activity, alpha-N-acylaminoacid hydrolase activity, amido acid deacylase activity, benzamidase activity, hippurase activity, histozyme activity, long acyl amidoacylase activity, short acyl amidoacylase activity